{
  "term_id": "GO:0005634",
  "gene_name": "Nuclear apoptosis-inducing factor 1",
  "gene_symbol": "NAIF1",
  "gene": "UniProtKB:Q69YI7",
  "term_label": "nucleus"
}